{
  "term_label": "protein kinase binding",
  "gene_symbol": "PRKAG1",
  "term_id": "GO:0019901",
  "gene_name": "5'-AMP-activated protein kinase subunit gamma-1",
  "gene": "UniProtKB:P54619"
}